{
  "term_label": "Golgi apparatus",
  "gene_symbol": "FAM20A",
  "gene": "UniProtKB:Q96MK3",
  "gene_name": "Pseudokinase FAM20A",
  "term_id": "GO:0005794"
}